{
  "term_label": "DNA replication",
  "gene_name": "ATP-dependent DNA helicase Q5",
  "gene": "UniProtKB:O94762",
  "gene_symbol": "RECQL5",
  "term_id": "GO:0006260"
}